{
  "gene_symbol": "ZNF707",
  "term_label": "DNA-binding transcription factor activity",
  "gene_name": "Zinc finger protein 707",
  "term_id": "GO:0003700",
  "gene": "UniProtKB:Q96C28"
}